detection of nuclear:cytoplasmic ratio [GO:0016475] (biological process) Definition: The process in which the size of the nucleus with respect to its cytoplasm is sensed by a cell. Sources: GOC:jl Also known as: interpretation of nuclear:cytoplasmic ratio, sensing of nuclear:cytoplasmic ratio Relationships: is a type of GO:0071495; is part of cell growth [GO:0016049]